{
  "gene_symbol": "CAV2",
  "term_label": "cytoplasmic vesicle",
  "gene_name": "Caveolin-2",
  "gene": "UniProtKB:P51636",
  "term_id": "GO:0031410"
}